negative regulation of renal albumin absorption [GO:2000533] (biological process) Relationships: is a type of negative regulation of multicellular organismal process [GO:0051241]; is a type of GO:2000532; negatively regulates renal albumin absorption [GO:0097018] Definition: Any process that stops, prevents or reduces the frequency, rate or extent of renal albumin absorption. Sources: GOC:obol, GOC:yaf